dense core granule membrane [GO:0032127] (cellular component) Relationships: is a type of GO:0030667; is part of dense core granule [GO:0031045] Sources: GOC:mah Subtypes: neuronal dense core vesicle membrane [GO:0099012] Also known as: dense core vesicle membrane Definition: The lipid bilayer surrounding a dense core granule.